{
  "term_label": "intracellular sodium ion homeostasis",
  "gene": "UniProtKB:P54709",
  "gene_symbol": "ATP1B3",
  "term_id": "GO:0006883",
  "gene_name": "Sodium_potassium-transporting ATPase subunit beta-3"
}